{
  "gene_symbol": "CCR7",
  "gene": "UniProtKB:P32248",
  "gene_name": "C-C chemokine receptor type 7",
  "term_label": "chemokine (C-C motif) ligand 19 binding",
  "term_id": "GO:0035757"
}